mitotic actomyosin contractile ring, proximal layer [GO:0120104] (cellular component) Also known as: actomyosin contractile ring, proximal layer References: PMID:28914606 Sources: GOC:krc, GOC:vw Definition: The region of the mitotic actomyosin ring adjacent to the plasma membrane where membrane bound scaffolds are located. Relationships: is a type of cellular anatomical structure [GO:0110165]; is part of mitotic actomyosin contractile ring [GO:0110085]